{
  "term_label": "GABA-ergic synapse",
  "gene_name": "SLIT and NTRK-like protein 3",
  "term_id": "GO:0098982",
  "gene": "UniProtKB:O94933",
  "gene_symbol": "SLITRK3"
}